{
  "gene": "UniProtKB:P0CAP1",
  "term_label": "Unknown biological process",
  "term_id": "UNKNOWN:0002",
  "gene_name": "Myocardial zonula adherens protein",
  "gene_symbol": "MYZAP"
}